{
  "term_id": "GO:0006355",
  "term_label": "regulation of DNA-templated transcription",
  "gene_name": "Protein lin-54 homolog",
  "gene_symbol": "LIN54",
  "gene": "UniProtKB:Q6MZP7"
}